{
  "gene_symbol": "FAM66E",
  "term_label": "Unknown molecular function",
  "term_id": "UNKNOWN:0001",
  "gene": "UniProtKB:P0C841",
  "gene_name": "Putative protein FAM66E"
}